{
  "gene": "UniProtKB:Q6VVB1",
  "gene_symbol": "NHLRC1",
  "term_label": "ubiquitin protein ligase activity",
  "term_id": "GO:0061630",
  "gene_name": "E3 ubiquitin-protein ligase NHLRC1"
}